{
  "gene": "UniProtKB:A6NKD9",
  "term_label": "Unknown molecular function",
  "gene_name": "Coiled-coil domain-containing protein 85C",
  "term_id": "UNKNOWN:0001",
  "gene_symbol": "CCDC85C"
}